{
  "term_label": "apical junction complex",
  "gene": "UniProtKB:A6NKD9",
  "term_id": "GO:0043296",
  "gene_name": "Coiled-coil domain-containing protein 85C",
  "gene_symbol": "CCDC85C"
}